type B pancreatic cell maturation [GO:0072560] (biological process) Definition: A developmental process, independent of morphogenetic (shape) change, that is required for a type B pancreatic cell to attain its fully functional state. A type B pancreatic cell is a cell located towards center of the islets of Langerhans that secretes insulin. Relationships: is a type of epithelial cell maturation [GO:0002070]; is part of GO:0003323 Also known as: pancreatic B cell maturation, pancreatic beta cell maturation Note: These processes continue to 60 DPA in Gossypium spp. Sources: CL:0000169, GOC:BHF